{
  "term_id": "GO:0004843",
  "gene_symbol": "ATXN3L",
  "gene_name": "Ataxin-3-like protein",
  "term_label": "cysteine-type deubiquitinase activity",
  "gene": "UniProtKB:Q9H3M9"
}